{
  "gene_name": "Gastric inhibitory polypeptide",
  "term_label": "glucagon receptor binding",
  "gene": "UniProtKB:P09681",
  "term_id": "GO:0031769",
  "gene_symbol": "GIP"
}